{
  "gene_symbol": "NDUFA8",
  "gene": "UniProtKB:P51970",
  "gene_name": "NADH dehydrogenase [ubiquinone] 1 alpha subcomplex subunit 8",
  "term_id": "GO:0045271",
  "term_label": "respiratory chain complex I"
}